{
  "term_label": "receptor complex",
  "gene": "UniProtKB:Q8NI17",
  "gene_name": "Interleukin-31 receptor subunit alpha",
  "gene_symbol": "IL31RA",
  "term_id": "GO:0043235"
}